response to iloperidone [GO:0036287] (biological process) Definition: Any process that results in a change in state or activity of a cell or an organism (in terms of movement, secretion, enzyme production, gene expression, etc.) as a result of an iloperidone stimulus. Note: Note that this term is in the subset of terms that should not be used for direct manual annotation of gene products. It was created to be used for cross-referencing by other ontologies. Direct annotations to this term may be amended during annotation QC. Relationships: is a type of response to ether [GO:0045472]; is a type of response to monoamine [GO:0071867]; is a type of response to ketone [GO:1901654] Sources: GOC:hp